central B cell tolerance induction [GO:0002510] (biological process) Relationships: is a type of central tolerance induction [GO:0002508]; is_a B cell tolerance induction [GO:0002514] Regulation: regulated by regulation of central B cell tolerance induction [GO:0002895]; negatively regulated by GO:0002896; positively regulated by positive regulation of central B cell tolerance induction [GO:0002897] Definition: Tolerance induction of B cells in the bone marrow. Also known as: central B lymphocyte tolerance induction, central B-cell tolerance induction, central B-lymphocyte tolerance induction References: PMID:16460922 Sources: GOC:jal